{
  "gene_name": "CEP295 N-terminal-like protein",
  "gene_symbol": "CEP295NL",
  "term_id": "GO:0005829",
  "gene": "UniProtKB:Q96MC4",
  "term_label": "cytosol"
}